cytoplasmic side of Golgi membrane [GO:0098548] (cellular component) Sources: GOC:ab, GOC:dos Relationships: is a type of GO:0098562; is part of GO:0000139 Definition: The side (leaflet) of the Golgi membrane that faces the cytoplasm.